cellular response to L-ascorbic acid [GO:0071298] (biological process) Definition: Any process that results in a change in state or activity of a cell (in terms of movement, secretion, enzyme production, gene expression, etc.) as a result of an L-ascorbic acid (vitamin C) stimulus. Relationships: is a type of response to L-ascorbic acid [GO:0033591]; is a type of cellular response to vitamin [GO:0071295]; is a type of cellular response to monosaccharide stimulus [GO:0071326] Sources: GOC:mah Also known as: cellular response to ascorbic acid, cellular response to L-ascorbate, cellular response to vitamin C